{
  "term_label": "dense core granule priming",
  "gene_symbol": "UNC13B",
  "gene": "UniProtKB:O14795",
  "gene_name": "Protein unc-13 homolog B",
  "term_id": "GO:0061789"
}